{
  "term_label": "Golgi membrane",
  "term_id": "GO:0000139",
  "gene_name": "Calcium-transporting ATPase type 2C member 1",
  "gene": "UniProtKB:P98194",
  "gene_symbol": "ATP2C1"
}